{
  "term_id": "GO:0045664",
  "term_label": "regulation of neuron differentiation",
  "gene": "UniProtKB:Q9UM73",
  "gene_symbol": "ALK",
  "gene_name": "ALK tyrosine kinase receptor"
}